positive regulation of mitochondrial membrane permeability involved in apoptotic process [GO:1902110] (biological process) Also known as: positive regulation of mitochondrial membrane permeability involved in apoptotic cell death, positive regulation of mitochondrial membrane permeability involved in apoptotic programmed cell death, positive regulation of mitochondrial membrane permeability involved in programmed cell death by apoptosis, positive regulation of transport across mitochondrial membrane involved in apoptotic cell death, positive regulation of transport across mitochondrial membrane involved in apoptotic process, positive regulation of transport across mitochondrial membrane involved in apoptotic programmed cell death, positive regulation of transport across mitochondrial membrane involved in programmed cell death by apoptosis, mitochondrial membrane permeability transition involved in apoptosis, mitochondrial membrane permeability transition involved in apoptotic cell death, mitochondrial membrane permeability transition involved in apoptotic process, mitochondrial membrane permeability transition involved in apoptotic program, mitochondrial membrane permeability transition involved in apoptotic programmed cell death, mitochondrial membrane permeability transition involved in programmed cell death by apoptosis, mitochondrial membrane permeability transition involved in type I programmed cell death, mitochondrial membrane permeabilization involved in apoptosis, mitochondrial membrane permeabilization involved in apoptotic cell death, mitochondrial membrane permeabilization involved in apoptotic process, mitochondrial membrane permeabilization involved in apoptotic program, mitochondrial membrane permeabilization involved in apoptotic programmed cell death, mitochondrial membrane permeabilization involved in programmed cell death by apoptosis, mitochondrial membrane permeabilization involved in type I programmed cell death, mitochondrial permeability transition involved in apoptosis, mitochondrial permeability transition involved in apoptotic cell death, mitochondrial permeability transition involved in apoptotic process, mitochondrial permeability transition involved in apoptotic program, mitochondrial permeability transition involved in apoptotic programmed cell death, mitochondrial permeability transition involved in programmed cell death by apoptosis, mitochondrial permeability transition involved in type I programmed cell death, positive regulation of mitochondrial membrane permeability involved in apoptosis, positive regulation of mitochondrial membrane permeability involved in apoptotic program, positive regulation of mitochondrial membrane permeability involved in type I programmed cell death, positive regulation of transport across mitochondrial membrane involved in apoptosis, positive regulation of transport across mitochondrial membrane involved in apoptotic program, positive regulation of transport across mitochondrial membrane involved in type I programmed cell death, mitochondrial membrane permeability transition involved in signaling (initiator) caspase activity, mitochondrial membrane permeabilization involved in signaling (initiator) caspase activity, mitochondrial permeability transition involved in signaling (initiator) caspase activity, positive regulation of mitochondrial membrane permeability involved in signaling (initiator) caspase activity, positive regulation of transport across mitochondrial membrane involved in signaling (initiator) caspase activity Relationships: is a type of GO:1902108; is a type of mitochondrial outer membrane permeabilization involved in programmed cell death [GO:1902686] References: PMID:19168129 Sources: GOC:TermGenie, GOC:mtg_apoptosis, GOC:pm Definition: Any positive regulation of mitochondrial membrane permeability that is involved in apoptotic process. Note: Individual components of the mitochondrial permeability transition pore complex, such as the voltage-dependent anion channel (VDAC), the adenine nucleotide translocase (ANT) and cyclophilin-D (CyP-D), are involved in this process. Subtypes: mitochondrial outer membrane permeabilization [GO:0097345]